pyridinol guanylyltransferase activity [GO:0160298] (molecular function) References: PMID:24249552 Definition: Catalysis of the reaction: 6-carboxymethyl-3,5-dimethyl-4-hydroxypyridin-2-ol + GTP + H+ = guanylylpyridinol + diphosphate. Relationships: is a type of guanylyltransferase activity [GO:0070568]